{
  "gene": "UniProtKB:O43301",
  "gene_symbol": "HSPA12A",
  "gene_name": "Heat shock 70 kDa protein 12A",
  "term_label": "Unknown molecular function",
  "term_id": "UNKNOWN:0001"
}